{
  "gene_name": "Choline transporter-like protein 2",
  "term_label": "transmembrane transport",
  "gene_symbol": "SLC44A2",
  "term_id": "GO:0055085",
  "gene": "UniProtKB:Q8IWA5"
}